phagocytic cup base [GO:0097204] (cellular component) Relationships: is a type of cellular anatomical structure [GO:0110165]; is part of phagocytic cup [GO:0001891] References: PMID:20200225 Sources: GOC:pf Definition: The older part of the phagocytic cup where the actin cytoskeleton disassembles, allowing early incoming and outgoing vesicular trafficking.